{
  "gene": "UniProtKB:Q14183",
  "gene_symbol": "DOC2A",
  "term_label": "calcium-dependent activation of synaptic vesicle fusion",
  "term_id": "GO:0099502",
  "gene_name": "Double C2-like domain-containing protein alpha"
}